{
  "gene": "UniProtKB:O43505",
  "term_label": "protein O-linked glycosylation via mannose",
  "gene_name": "Beta-1,4-glucuronyltransferase 1",
  "term_id": "GO:0035269",
  "gene_symbol": "B4GAT1"
}